{
  "term_id": "GO:0009897",
  "term_label": "external side of plasma membrane",
  "gene": "UniProtKB:P16871",
  "gene_symbol": "IL7R",
  "gene_name": "Interleukin-7 receptor subunit alpha"
}